{
  "term_id": "GO:0102102",
  "gene_name": "Carnosine synthase 1",
  "term_label": "homocarnosine synthase activity",
  "gene_symbol": "CARNS1",
  "gene": "UniProtKB:A5YM72"
}